{
  "gene_name": "MAP kinase-interacting serine_threonine-protein kinase 1",
  "gene_symbol": "MKNK1",
  "term_id": "GO:0009931",
  "term_label": "calcium-dependent protein serine/threonine kinase activity",
  "gene": "UniProtKB:Q9BUB5"
}